{
  "term_label": "cytoplasm",
  "gene_symbol": "DUSP6",
  "term_id": "GO:0005737",
  "gene": "UniProtKB:Q16828",
  "gene_name": "Dual specificity protein phosphatase 6"
}